positive regulation of myofibroblast contraction [GO:1904330] (biological process) Also known as: positive regulation of MF contraction, positive regulation of MFB contraction, up regulation of MF contraction, up regulation of MFB contraction, up regulation of myofibroblast contraction, up-regulation of MF contraction, up-regulation of MFB contraction, up-regulation of myofibroblast contraction, upregulation of MF contraction, upregulation of MFB contraction, upregulation of myofibroblast contraction, activation of MF contraction, activation of MFB contraction, activation of myofibroblast contraction Definition: Any process that activates or increases the frequency, rate or extent of myofibroblast contraction. Relationships: is a type of positive regulation of actin filament-based movement [GO:1903116]; is_a regulation of myofibroblast contraction [GO:1904328]; positively regulates myofibroblast contraction [GO:1990764] References: PMID:19239477 Sources: GOC:TermGenie, GO_REF:0000058